olfactory sociosexual communication [GO:0120318] (biological process) Relationships: is_a behavior [GO:0007610]; is a type of biological process involved in intraspecies interaction between organisms [GO:0051703] References: PMID:17935991 Sources: GOC:krc Definition: The use of external chemical cues called pheromones to send social and sexual information between members of the same species, leading to specific behavioral responses. Pheromones may be detected by two olfactory sensory circuits, the main olfactory pathway and the vomeronasal system. Note: Behavior such as predation which involves members of different species is not social. Communication between members of different species is also not social behavior.